{
  "gene_symbol": "TMED9",
  "term_id": "UNKNOWN:0001",
  "gene": "UniProtKB:Q9BVK6",
  "term_label": "Unknown molecular function",
  "gene_name": "Transmembrane emp24 domain-containing protein 9"
}